3-demethylubiquinol 3-O-methyltransferase activity [GO:0061542] (molecular function) Note: Note that the polyprenyl sidechain substrate for this reaction has a different number of prenyl units in different organisms (for example, ubiquinone-6 in Saccharomyces, ubiquinone- 9 in rat and ubiquinone-10 in human), and thus the natural substrate for the enzymes from different organisms has a different number of prenyl units. However, the enzyme usually shows a low degree of specificity regarding the number of prenyl units. Also known as: 3-demethylubiquinol-n 3-O-methyltransferase activity, 2-octaprenyl-3-methyl-5-hydroxy-6-methoxy-1,4-benzoquinone methyltransferase, 5-demethylubiquinone-10 methyltransferase, 5-demethylubiquinone-9 methyltransferase, OMHMB-methyltransferase, S-adenosyl-L-methionine:2-octaprenyl-3-methyl-5-hydroxy-6-methoxy-1,4-benzoquinone-O-methyltransferase Relationships: is a type of O-methyltransferase activity [GO:0008171]; is a type of S-adenosylmethionine-dependent methyltransferase activity [GO:0008757]; is part of ubiquinone biosynthetic process [GO:0006744] References: PMID:10777520, PMID:23190198 Sources: RHEA:44380 Definition: Catalysis of the reaction: a 3-demethylubiquinol + S-adenosyl-L-methionine = a ubiquinol + S-adenosyl-L-homocysteine + H+.